{
  "gene_symbol": "PAX5",
  "term_id": "GO:0007423",
  "gene_name": "Paired box protein Pax-5",
  "term_label": "sensory organ development",
  "gene": "UniProtKB:Q02548"
}